{
  "term_id": "GO:0090141",
  "gene_name": "Serine_threonine-protein kinase PINK1, mitochondrial",
  "term_label": "positive regulation of mitochondrial fission",
  "gene": "UniProtKB:Q9BXM7",
  "gene_symbol": "PINK1"
}